floral organ formation [GO:0048449] (biological process) Definition: The process that gives rise to floral organs. This process pertains to the initial formation of a structure from unspecified parts. Relationships: is a type of developmental process involved in reproduction [GO:0003006]; is a type of plant organ formation [GO:1905393]; BFO_0000050 floral organ morphogenesis [GO:0048444] Sources: GOC:PO_curators, GOC:jid, PO:0025395 Subtypes: petal formation [GO:0048451], sepal formation [GO:0048453], stamen formation [GO:0048455], carpel formation [GO:0048462]